{
  "term_id": "GO:0043161",
  "gene_symbol": "PRAMEF4",
  "gene": "UniProtKB:O60810",
  "gene_name": "PRAME family member 4",
  "term_label": "proteasome-mediated ubiquitin-dependent protein catabolic process"
}